{
  "gene_symbol": "BMP15",
  "gene_name": "Bone morphogenetic protein 15",
  "gene": "UniProtKB:O95972",
  "term_id": "GO:0005125",
  "term_label": "cytokine activity"
}